{
  "term_label": "Unknown molecular function",
  "gene_symbol": "DPM3",
  "gene": "UniProtKB:Q9P2X0",
  "gene_name": "Dolichol-phosphate mannosyltransferase subunit 3",
  "term_id": "UNKNOWN:0001"
}